{
  "gene": "UniProtKB:Q8NGZ3",
  "term_id": "GO:0016020",
  "gene_name": "Olfactory receptor 13G1",
  "gene_symbol": "OR13G1",
  "term_label": "membrane"
}